phytoalexin biosynthetic process [GO:0052315] (biological process) Definition: The chemical reactions and pathways resulting in the formation of phytoalexins, any of a range of substances produced by plants as part of their defense response. References: PMID:22209038, PMID:3882051 Sources: Wikipedia:Phytoalexin Also known as: phytoalexin biosynthesis Relationships: is a type of toxin biosynthetic process [GO:0009403]; is a type of phytoalexin metabolic process [GO:0052314] Subtypes: indole phytoalexin biosynthetic process [GO:0009700], isoflavonoid phytoalexin biosynthetic process [GO:0009701], flavonoid phytoalexin biosynthetic process [GO:0009716], diterpene phytoalexin biosynthetic process [GO:0051502] Regulation: positively regulated by positive regulation of phytoalexin biosynthetic process [GO:0052322]